Yae1-Lto1 complex [GO:0062092] (cellular component) Definition: A cytosolic complex that functions as an substrate-specific adaptor, linking the cytosolic iron-sulfur protein assembly (CIA) targeting complex to apo-Rli1p, an ABC protein involved in ribosome recycling, facilitating Fe-S cluster insertion and the maturation of the Rli1p. References: PMID:26182403 Relationships: is a type of protein-containing complex [GO:0032991]; is part of cytosol [GO:0005829]